lincomycin biosynthetic process [GO:1901774] (biological process) Also known as: lincomycin anabolism, lincomycin biosynthesis, lincomycin formation, lincomycin synthesis Definition: The chemical reactions and pathways resulting in the formation of lincomycin. References: PMID:8577249 Sources: GOC:TermGenie, GOC:yaf, MetaCyc:PWY-6955, UniPathway:UPA00161 Relationships: is a type of S-glycoside biosynthetic process [GO:0016144]; is a type of modified amino acid biosynthetic process [GO:0042398]; is a type of amide biosynthetic process [GO:0043604]